{
  "term_id": "GO:0004674",
  "gene_symbol": "DAPK3",
  "gene_name": "Death-associated protein kinase 3",
  "gene": "UniProtKB:O43293",
  "term_label": "protein serine/threonine kinase activity"
}